{
  "gene_symbol": "ZC3H12D",
  "gene_name": "Probable ribonuclease ZC3H12D",
  "term_label": "RNA endonuclease activity",
  "gene": "UniProtKB:A2A288",
  "term_id": "GO:0004521"
}